intermediate layer of mitotic spindle pole body [GO:0061498] (cellular component) Relationships: is a type of GO:0005821; is part of mitotic spindle pole body [GO:0044732] Sources: GOC:dph Definition: Structure between the central and outer plaques of the mitotic spindle pole body.